{
  "term_id": "GO:0030334",
  "term_label": "regulation of cell migration",
  "gene_name": "Plexin-B2",
  "gene": "UniProtKB:O15031",
  "gene_symbol": "PLXNB2"
}